{
  "gene": "UniProtKB:Q08AI8",
  "term_label": "Unknown molecular function",
  "term_id": "UNKNOWN:0001",
  "gene_name": "Protein mab-21-like 4",
  "gene_symbol": "MAB21L4"
}